{
  "gene_symbol": "TPX2",
  "gene_name": "Targeting protein for Xklp2",
  "term_label": "mitotic spindle assembly",
  "term_id": "GO:0090307",
  "gene": "UniProtKB:Q9ULW0"
}